2-carboxy-D-arabinitol-1-phosphatase activity [GO:0047538] (molecular function) Also known as: 2-carboxy-D-arabinitol 1-phosphate phosphohydrolase activity, 2-carboxy-D-arabinitol-1-phosphate 1-phosphohydrolase activity, 2-carboxyarabinitol 1-phosphatase activity Relationships: is a type of phosphatase activity [GO:0016791] Definition: Catalysis of the reaction: 2-carboxy-D-arabinitol 1-phosphate + H2O = 2-carboxy-D-arabinitol + phosphate. Sources: EC:3.1.3.63, RHEA:17837